{
  "gene_symbol": "PLXNC1",
  "gene_name": "Plexin-C1",
  "term_label": "synapse assembly",
  "term_id": "GO:0007416",
  "gene": "UniProtKB:O60486"
}